{
  "term_label": "endoplasmic reticulum",
  "term_id": "GO:0005783",
  "gene_symbol": "POMT1",
  "gene_name": "Protein O-mannosyl-transferase 1",
  "gene": "UniProtKB:Q9Y6A1"
}